{
  "gene_symbol": "ST14",
  "gene": "UniProtKB:Q9Y5Y6",
  "gene_name": "Suppressor of tumorigenicity 14 protein",
  "term_label": "serine-type peptidase activity",
  "term_id": "GO:0008236"
}